{
  "term_label": "cortical actin cytoskeleton organization",
  "gene_name": "Nck-associated protein 1-like",
  "gene_symbol": "NCKAP1L",
  "term_id": "GO:0030866",
  "gene": "UniProtKB:P55160"
}